{
  "gene": "UniProtKB:Q12841",
  "gene_name": "Follistatin-related protein 1",
  "gene_symbol": "FSTL1",
  "term_id": "UNKNOWN:0001",
  "term_label": "Unknown molecular function"
}